{
  "gene_symbol": "ADGRF1",
  "gene_name": "Adhesion G-protein coupled receptor F1",
  "gene": "UniProtKB:Q5T601",
  "term_id": "GO:0031175",
  "term_label": "neuron projection development"
}